{
  "gene_name": "ATP synthase subunit epsilon-like protein, mitochondrial",
  "gene": "UniProtKB:Q5VTU8",
  "term_label": "proton motive force-driven mitochondrial ATP synthesis",
  "gene_symbol": "ATP5F1EP2",
  "term_id": "GO:0042776"
}